regulation of ARF protein signal transduction [GO:0032012] (BP) Subtypes: GO:0032013, positive regulation of ARF protein signal transduction [GO:0032014] Relationships: is a type of regulation of small GTPase mediated signal transduction [GO:0051056]; regulates ARF protein signal transduction [GO:0032011] Sources: GOC:mah Definition: Any process that modulates the frequency, rate or extent of ARF protein signal transduction.